{
  "gene_symbol": "MAGEB1",
  "term_id": "GO:0005634",
  "gene": "UniProtKB:P43366",
  "term_label": "nucleus",
  "gene_name": "Melanoma-associated antigen B1"
}